{
  "gene": "UniProtKB:O60858",
  "gene_name": "E3 ubiquitin-protein ligase TRIM13",
  "gene_symbol": "TRIM13",
  "term_label": "innate immune response",
  "term_id": "GO:0045087"
}